{
  "gene_name": "Sulfotransferase 1C2",
  "term_id": "GO:0004062",
  "gene": "UniProtKB:O00338",
  "term_label": "aryl sulfotransferase activity",
  "gene_symbol": "SULT1C2"
}